C21-steroid hormone metabolic process [GO:0008207] (biological process) Also known as: C21-steroid hormone metabolism Relationships: is_a steroid metabolic process [GO:0008202]; is a type of hormone metabolic process [GO:0042445] Definition: The chemical reactions and pathways involving C21-steroid hormones, steroid compounds containing 21 carbons which function as hormones. Subtypes: C21-steroid hormone biosynthetic process [GO:0006700], C21-steroid hormone catabolic process [GO:0008208], aldosterone metabolic process [GO:0032341], progesterone metabolic process [GO:0042448] Sources: GOC:ai